{
  "term_label": "sequence-specific DNA binding",
  "gene_symbol": "HLX",
  "term_id": "GO:0043565",
  "gene_name": "H2.0-like homeobox protein",
  "gene": "UniProtKB:Q14774"
}